{
  "gene_symbol": "GSN-AS1",
  "term_id": "UNKNOWN:0001",
  "gene_name": "Putative uncharacterized protein GSN-AS1",
  "term_label": "Unknown molecular function",
  "gene": "UniProtKB:Q9NRJ2"
}